{
  "gene": "UniProtKB:P20941",
  "gene_name": "Phosducin",
  "term_label": "Unknown molecular function",
  "term_id": "UNKNOWN:0001",
  "gene_symbol": "PDC"
}